{
  "term_id": "GO:0007004",
  "gene": "UniProtKB:Q15185",
  "term_label": "telomere maintenance via telomerase",
  "gene_symbol": "PTGES3",
  "gene_name": "Prostaglandin E synthase 3"
}